{
  "gene_name": "Toll-like receptor 1",
  "term_id": "GO:0002224",
  "gene_symbol": "TLR1",
  "gene": "UniProtKB:Q15399",
  "term_label": "toll-like receptor signaling pathway"
}